{
  "gene_symbol": "MT-ATP6",
  "term_id": "GO:0046933",
  "gene": "UniProtKB:P00846",
  "gene_name": "ATP synthase subunit a",
  "term_label": "proton-transporting ATP synthase activity, rotational mechanism"
}